{
  "term_id": "UNKNOWN:0003",
  "gene_name": "Inactive ribonuclease-like protein 9",
  "term_label": "Unknown cellular component",
  "gene_symbol": "RNASE9",
  "gene": "UniProtKB:P60153"
}